{
  "gene_symbol": "PKMYT1",
  "term_id": "GO:0051321",
  "term_label": "meiotic cell cycle",
  "gene_name": "Membrane-associated tyrosine- and threonine-specific cdc2-inhibitory kinase",
  "gene": "UniProtKB:Q99640"
}